{
  "gene_symbol": "MX1",
  "term_label": "GTPase activity",
  "gene_name": "Interferon-induced GTP-binding protein Mx1",
  "gene": "UniProtKB:P20591",
  "term_id": "GO:0003924"
}